negative regulation of collagen metabolic process [GO:0010713] (biological process) Sources: GOC:dph, GOC:tb Definition: Any process that decreases the frequency, rate or extent of the chemical reactions and pathways resulting in the metabolism of collagen, any of a group of fibrous proteins of very high tensile strength that form the main component of connective tissue in animals. Subtypes: negative regulation of collagen catabolic process [GO:0010711], GO:0032966 Relationships: is a type of GO:0009892; is a type of GO:0010712; negatively regulates collagen metabolic process [GO:0032963]